{
  "gene": "UniProtKB:Q86Y79",
  "gene_symbol": "PTRH1",
  "term_label": "peptidyl-tRNA hydrolase activity",
  "gene_name": "Peptidyl-tRNA hydrolase",
  "term_id": "GO:0004045"
}